{
  "term_label": "cytoskeleton",
  "term_id": "GO:0005856",
  "gene_name": "Serine_threonine-protein kinase MRCK alpha",
  "gene_symbol": "CDC42BPA",
  "gene": "UniProtKB:Q5VT25"
}